{
  "term_label": "Unknown biological process",
  "term_id": "UNKNOWN:0002",
  "gene": "UniProtKB:Q8IZJ6",
  "gene_name": "Inactive L-threonine 3-dehydrogenase, mitochondrial",
  "gene_symbol": "TDH"
}